{
  "gene_name": "GTP-binding protein Di-Ras2",
  "term_id": "GO:0003924",
  "gene": "UniProtKB:Q96HU8",
  "term_label": "GTPase activity",
  "gene_symbol": "DIRAS2"
}